{
  "term_id": "GO:0005634",
  "gene_name": "Apoptosis-associated speck-like protein containing a CARD",
  "gene": "UniProtKB:Q9ULZ3",
  "term_label": "nucleus",
  "gene_symbol": "PYCARD"
}